{
  "term_label": "DNA-binding transcription factor activity, RNA polymerase II-specific",
  "gene": "UniProtKB:Q5T1R4",
  "term_id": "GO:0000981",
  "gene_name": "Transcription factor HIVEP3",
  "gene_symbol": "HIVEP3"
}